negative regulation of cardioblast differentiation [GO:0051892] (biological process) Relationships: is a type of regulation of cardioblast differentiation [GO:0051890]; is a type of negative regulation of cardiocyte differentiation [GO:1905208]; is a type of negative regulation of stem cell differentiation [GO:2000737]; negatively regulates cardioblast differentiation [GO:0010002] Sources: GOC:ai Definition: Any process that stops, prevents, or reduces the frequency, rate or extent of cardioblast differentiation, the process in which a relatively unspecialized mesodermal cell acquires the specialized structural and/or functional features of a cardioblast. A cardioblast is a cardiac precursor cell. It is a cell that has been committed to a cardiac fate, but will undergo more cell division rather than terminally differentiating. Also known as: down regulation of cardioblast differentiation, down-regulation of cardioblast differentiation, downregulation of cardioblast differentiation, inhibition of cardioblast differentiation Subtypes: negative regulation of cardioblast cell fate specification [GO:0009997], GO:2000691